{
  "term_id": "GO:2000134",
  "gene_name": "Retinoblastoma-like protein 1",
  "gene_symbol": "RBL1",
  "term_label": "negative regulation of G1/S transition of mitotic cell cycle",
  "gene": "UniProtKB:P28749"
}